positive regulation of fatty acid beta-oxidation by octopamine signaling pathway [GO:1904122] (biological process) Also known as: up regulation of fatty acid beta-oxidation by octopamine signaling pathway, up-regulation of fatty acid beta-oxidation by octopamine signaling pathway, upregulation of fatty acid beta-oxidation by octopamine signaling pathway, activation of fatty acid beta-oxidation by octopamine signaling pathway, stimulation of fatty acid beta-oxidation by octopamine signaling pathway Relationships: is a type of positive regulation of fatty acid beta-oxidation [GO:0032000]; is a type of GO:0071927 References: PMID:24120942 Sources: GOC:TermGenie, GOC:dph, GOC:kmv, GO_REF:0000063 Definition: An octopamine signaling pathway that results in positive regulation of fatty acid beta-oxidation.